{
  "gene": "UniProtKB:Q9BU20",
  "term_label": "ciliary basal body",
  "gene_name": "Ciliogenesis and planar polarity effector 2",
  "gene_symbol": "CPLANE2",
  "term_id": "GO:0036064"
}